{
  "gene": "UniProtKB:O75122",
  "term_label": "cytoplasmic microtubule",
  "term_id": "GO:0005881",
  "gene_name": "CLIP-associating protein 2",
  "gene_symbol": "CLASP2"
}